outward migration of deep nuclear neurons [GO:0021947] (biological process) Relationships: is a type of GO:0001764; is a type of cell migration in hindbrain [GO:0021535]; is part of GO:0021946 Definition: The directed movement of a deep nuclear neuron from their ventrolateral origin to a rostrodorsal region of the cerebellar plate. References: PMID:15157725 Sources: GOC:cls, GOC:dgh, GOC:dph, GOC:jid, GO_REF:0000021